{
  "term_id": "GO:0031681",
  "term_label": "G-protein beta-subunit binding",
  "gene": "UniProtKB:Q96D21",
  "gene_name": "GTP-binding protein Rhes",
  "gene_symbol": "RASD2"
}